{
  "gene_name": "Beta-defensin 133",
  "gene_symbol": "DEFB133",
  "term_id": "GO:0042056",
  "term_label": "chemoattractant activity",
  "gene": "UniProtKB:Q30KQ1"
}